{
  "gene_name": "Peroxisomal biogenesis factor 3",
  "gene_symbol": "PEX3",
  "term_label": "peroxisomal membrane",
  "gene": "UniProtKB:P56589",
  "term_id": "GO:0005778"
}